{
  "term_label": "Unknown cellular component",
  "gene_name": "Group XIIB secretory phospholipase A2-like protein",
  "term_id": "UNKNOWN:0003",
  "gene": "UniProtKB:Q9BX93",
  "gene_symbol": "PLA2G12B"
}